{
  "gene_name": "Zinc finger protein 528",
  "term_label": "RNA polymerase II cis-regulatory region sequence-specific DNA binding",
  "gene_symbol": "ZNF528",
  "term_id": "GO:0000978",
  "gene": "UniProtKB:Q3MIS6"
}